L-dopa metabolic process [GO:1903184] (biological process) References: PMID:8822146 Sources: GOC:PARL, GOC:TermGenie, GOC:bf, GO_REF:0000068 Subtypes: L-dopa biosynthetic process [GO:1903185] Also known as: L-dopa metabolism Definition: The chemical reactions and pathways involving L-dopa. Relationships: is a type of modified amino acid metabolic process [GO:0006575]; is a type of aromatic amino acid metabolic process [GO:0009072]; is a type of L-amino acid metabolic process [GO:0170033]; is a type of non-proteinogenic amino acid metabolic process [GO:0170041]